secondary-alcohol oxidase activity [GO:0033714] (molecular function) Definition: Catalysis of the reaction: secondary alcohol + O2 = H2O2 + ketone. Relationships: is a type of GO:0016899 Sources: EC:1.1.3.18, RHEA:23180 Also known as: polyvinyl alcohol oxidase activity, secondary alcohol oxidase activity, secondary-alcohol:oxygen oxidoreductase activity